{
  "gene_symbol": "TTC9C",
  "term_id": "UNKNOWN:0003",
  "term_label": "Unknown cellular component",
  "gene": "UniProtKB:Q8N5M4",
  "gene_name": "Tetratricopeptide repeat protein 9C"
}